scymnol sulfotransferase activity [GO:0033874] (molecular function) Sources: EC:2.8.2.32, RHEA:15477 Definition: Catalysis of the reaction: 3'-phospho-5'-adenylyl sulfate + 5beta-scymnol = 5beta-scymnol sulfate + adenosine 3',5'-diphosphate + H+. Relationships: is a type of sulfotransferase activity [GO:0008146]